{
  "gene": "UniProtKB:Q8IXM2",
  "term_label": "NURF complex",
  "gene_name": "Chromatin complexes subunit BAP18",
  "gene_symbol": "BAP18",
  "term_id": "GO:0016589"
}